guanosine pentaphosphate metabolic process [GO:0015972] (biological process) Relationships: is a type of purine ribonucleotide metabolic process [GO:0009150]; is a type of purine ribonucleoside bisphosphate metabolic process [GO:0034035] Sources: GOC:ai Definition: The chemical reactions and pathways involving guanine pentaphosphate (5'-pppGpp-3'), a derivative of guanine riboside with five phosphates. Also known as: guanosine pentaphosphate (5'-pppGpp-3') metabolic process, guanosine pentaphosphate (5'-pppGpp-3') metabolism, guanosine pentaphosphate metabolism Subtypes: guanosine pentaphosphate biosynthetic process [GO:0015973], guanosine pentaphosphate catabolic process [GO:0015974]